{
  "gene": "UniProtKB:Q6IFN5",
  "gene_symbol": "OR7E24",
  "term_label": "signal transduction",
  "term_id": "GO:0007165",
  "gene_name": "Olfactory receptor 7E24"
}